{
  "term_id": "GO:0019221",
  "gene": "UniProtKB:Q9UHA7",
  "gene_symbol": "IL36A",
  "term_label": "cytokine-mediated signaling pathway",
  "gene_name": "Interleukin-36 alpha"
}